pyridoxal phosphate biosynthetic process [GO:0042823] (biological process) Subtypes: pyridoxal 5'-phosphate salvage [GO:0009443], GO:0036001 Sources: GOC:jl Definition: The chemical reactions and pathways resulting in the formation of pyridoxal phosphate, pyridoxal phosphorylated at the hydroxymethyl group of C-5, the active form of vitamin B6. Relationships: is a type of GO:0042819; is a type of pyridoxal phosphate metabolic process [GO:0042822]; is a type of aldehyde biosynthetic process [GO:0046184]; is_a organophosphate biosynthetic process [GO:0090407] Also known as: active vitamin B6 biosynthesis, active vitamin B6 biosynthetic process, pyridoxal phosphate anabolism, pyridoxal phosphate biosynthesis, pyridoxal phosphate formation, pyridoxal phosphate synthesis